{
  "term_id": "GO:0050911",
  "term_label": "detection of chemical stimulus involved in sensory perception of smell",
  "gene": "UniProtKB:Q8NH80",
  "gene_symbol": "OR10D3",
  "gene_name": "Olfactory receptor 10D3"
}